{
  "gene": "UniProtKB:Q86U37",
  "term_label": "Unknown molecular function",
  "gene_name": "Uncharacterized protein encoded by LINC01551",
  "term_id": "UNKNOWN:0001",
  "gene_symbol": "LINC01551"
}